{
  "term_label": "regulation of transcription by RNA polymerase II",
  "gene_symbol": "ZBTB24",
  "term_id": "GO:0006357",
  "gene": "UniProtKB:O43167",
  "gene_name": "Zinc finger and BTB domain-containing protein 24"
}